ATP-dependent DNA (cytosine-5-)-methyltransferase activity [GO:0120328] (molecular function) Relationships: is a type of DNA (cytosine-5-)-methyltransferase activity [GO:0003886]; is a type of ATP-dependent activity, acting on DNA [GO:0008094] References: PMID:31955845, PMID:32437639 Sources: GOC:krc, RHEA:68984 Definition: Catalytic activity that acts to transfer a methyl group to a DNA molecule, driven by ATP hydrolysis.